{
  "term_id": "GO:0001228",
  "gene_symbol": "PBX4",
  "term_label": "DNA-binding transcription activator activity, RNA polymerase II-specific",
  "gene_name": "Pre-B-cell leukemia transcription factor 4",
  "gene": "UniProtKB:Q9BYU1"
}